retrograde transporter complex, Golgi to ER [GO:0061852] (cellular component) Definition: Transporter complex that recognises, binds and returns endoplasmic reticulum (ER) resident proteins that have trafficked to Golgi compartments. Targets proteins lacking the HDEL motif recognised by COPI-coated vesicles. Relationships: is_a transporter complex [GO:1990351] References: PMID:16093310 Sources: GOC:bhm Note: An example of this is ERV41 in Saccharomyces cerevisiae (Q04651) in PMID:16093310 (inferred from direct assay). Also known as: retrograde receptor complex, Golgi to ER, retrograde receptor complex, Golgi to endoplasmic reticulum, retrograde transporter complex, Golgi to endoplasmic reticulum, ERV41-ERV46 retrograde receptor complex